nucleobase-containing small molecule interconversion [GO:0015949] (biological process) Sources: GOC:mah, ISBN:0306444747, ISBN:0471394831 Relationships: is a type of nucleobase-containing small molecule metabolic process [GO:0055086] Subtypes: GO:0015950, pyrimidine nucleotide interconversion [GO:0015953], GO:0019686, pyrimidine nucleoside interconversion [GO:0019689] Definition: The chemical reactions and pathways by which a nucleobase, nucleoside or nucleotide small molecule is synthesized from another nucleobase, nucleoside or nucleotide small molecule.